{
  "gene": "UniProtKB:Q8WUF8",
  "gene_symbol": "ARB2A",
  "gene_name": "Cotranscriptional regulator FAM172A",
  "term_id": "GO:0031048",
  "term_label": "regulatory ncRNA-mediated heterochromatin formation"
}